{
  "gene_symbol": "CACFD1",
  "gene": "UniProtKB:Q9UGQ2",
  "gene_name": "Calcium channel flower homolog",
  "term_label": "Unknown cellular component",
  "term_id": "UNKNOWN:0003"
}